{
  "gene": "UniProtKB:O00512",
  "term_id": "GO:1990907",
  "term_label": "beta-catenin-TCF complex",
  "gene_symbol": "BCL9",
  "gene_name": "B-cell CLL_lymphoma 9 protein"
}